{
  "term_id": "GO:0000176",
  "gene_name": "Exosome complex component RRP45",
  "term_label": "nuclear exosome (RNase complex)",
  "gene_symbol": "EXOSC9",
  "gene": "UniProtKB:Q06265"
}